{
  "gene_symbol": "FAT4",
  "term_label": "cell-cell adhesion mediated by cadherin",
  "term_id": "GO:0044331",
  "gene_name": "Protocadherin Fat 4",
  "gene": "UniProtKB:Q6V0I7"
}